{
  "gene": "UniProtKB:Q9Y478",
  "term_label": "nucleus",
  "gene_symbol": "PRKAB1",
  "term_id": "GO:0005634",
  "gene_name": "5'-AMP-activated protein kinase subunit beta-1"
}